{
  "gene_symbol": "SNX2",
  "gene": "UniProtKB:O60749",
  "term_label": "endosome",
  "gene_name": "Sorting nexin-2",
  "term_id": "GO:0005768"
}